{
  "term_label": "cell surface",
  "gene_symbol": "ENPP1",
  "gene_name": "Ectonucleotide pyrophosphatase_phosphodiesterase family member 1",
  "term_id": "GO:0009986",
  "gene": "UniProtKB:P22413"
}